lactate transport [GO:0015727] (biological process) Subtypes: lactate transmembrane transport [GO:0035873] Relationships: is a type of monocarboxylic acid transport [GO:0015718]; is a type of GO:0015850 Sources: GOC:ai, ISBN:0198506732 Definition: The directed movement of lactate into, out of or within a cell, or between cells, by means of some agent such as a transporter or pore. Lactate is 2-hydroxypropanoate, CH3-CHOH-COOH; L(+)-lactate is formed by anaerobic glycolysis in animal tissues, and DL-lactate is found in sour milk, molasses and certain fruit juices.